{
  "gene": "UniProtKB:Q9NZW5",
  "term_label": "cell-cell junction",
  "term_id": "GO:0005911",
  "gene_symbol": "PALS2",
  "gene_name": "Protein PALS2"
}